(13S)-vitexifolin A synthase activity [GO:0062204] (molecular function) Relationships: is a type of GO:0016838 References: PMID:29315936 Sources: RHEA:40027 Definition: Catalysis of the reaction:9alpha-copalyl diphosphate + H2O = (13S)-vitexifolin A + diphosphate.